{
  "gene_symbol": "CHD9",
  "term_id": "UNKNOWN:0002",
  "gene_name": "Chromodomain-helicase-DNA-binding protein 9",
  "gene": "UniProtKB:Q3L8U1",
  "term_label": "Unknown biological process"
}